Set3 complex [GO:0034967] (cellular component) References: PMID:11711434 Sources: GOC:ds Definition: A histone deacetylase complex that is involved in transcriptional regulation. In S. cerevisiae, this complex consists of Set3p, Snt1p, Hos4p, Sif2p, Cpr1p, Hos2p, and Hst1p. Also known as: HDAC3 complex, SET3C Relationships: is a type of histone deacetylase complex [GO:0000118]; is part of nuclear chromosome [GO:0000228]; is part of chromatin [GO:0000785]